{
  "term_label": "Unknown cellular component",
  "gene_symbol": "KRTAP13-1",
  "term_id": "UNKNOWN:0003",
  "gene_name": "Keratin-associated protein 13-1",
  "gene": "UniProtKB:Q8IUC0"
}